{
  "gene_symbol": "PIM2",
  "term_id": "GO:0007346",
  "gene_name": "Serine_threonine-protein kinase pim-2",
  "gene": "UniProtKB:Q9P1W9",
  "term_label": "regulation of mitotic cell cycle"
}